positive regulation of phospholipase activity [GO:0010518] (biological process) Definition: Any process that increases the frequency, rate or extent of phospholipase activity, the hydrolysis of a phospholipid. Sources: GOC:BHF, GOC:dph, GOC:tb Relationships: is a type of regulation of phospholipase activity [GO:0010517]; is a type of GO:0060193; positively regulates phospholipase activity [GO:0004620]